{
  "gene_name": "Protein aurora borealis",
  "term_label": "cytoplasm",
  "gene_symbol": "BORA",
  "gene": "UniProtKB:Q6PGQ7",
  "term_id": "GO:0005737"
}